trichothecene 3-O-acetyltransferase activity [GO:0045462] (molecular function) References: PMID:10583973 Relationships: is a type of O-acetyltransferase activity [GO:0016413] Definition: Catalysis of the 3-O-acetylation of a trichothecene. Trichothecenes are sesquiterpene epoxide mycotoxins that act as potent inhibitors of eukaryotic protein synthesis.